{
  "gene": "UniProtKB:Q9H3H1",
  "gene_symbol": "TRIT1",
  "term_label": "mitochondrion",
  "term_id": "GO:0005739",
  "gene_name": "tRNA dimethylallyltransferase"
}